{
  "term_id": "GO:0007271",
  "gene_name": "Neuronal acetylcholine receptor subunit alpha-4",
  "gene_symbol": "CHRNA4",
  "term_label": "synaptic transmission, cholinergic",
  "gene": "UniProtKB:P43681"
}